{
  "gene": "UniProtKB:Q13003",
  "term_label": "synaptic transmission, glutamatergic",
  "term_id": "GO:0035249",
  "gene_symbol": "GRIK3",
  "gene_name": "Glutamate receptor ionotropic, kainate 3"
}